{
  "gene": "UniProtKB:Q71RC1",
  "term_id": "UNKNOWN:0002",
  "term_label": "Unknown biological process",
  "gene_name": "PP13850",
  "gene_symbol": "Q71RC1"
}